{
  "term_label": "regulation of cell cycle",
  "gene_symbol": "TXLNG",
  "gene": "UniProtKB:Q9NUQ3",
  "term_id": "GO:0051726",
  "gene_name": "Gamma-taxilin"
}